{
  "gene_symbol": "FZD4",
  "term_label": "plasma membrane",
  "term_id": "GO:0005886",
  "gene": "UniProtKB:Q9ULV1",
  "gene_name": "Frizzled-4"
}